{
  "gene_name": "Tetratricopeptide repeat protein 7A",
  "term_label": "phosphatidylinositol phosphate biosynthetic process",
  "term_id": "GO:0046854",
  "gene_symbol": "TTC7A",
  "gene": "UniProtKB:Q9ULT0"
}